{
  "gene_name": "G antigen 7",
  "gene_symbol": "GAGE7",
  "gene": "UniProtKB:O76087",
  "term_label": "Unknown molecular function",
  "term_id": "UNKNOWN:0001"
}